{
  "gene_symbol": "GPR50",
  "gene_name": "Melatonin-related receptor",
  "gene": "UniProtKB:Q13585",
  "term_id": "GO:0007186",
  "term_label": "G protein-coupled receptor signaling pathway"
}